{
  "gene_symbol": "DEFB118",
  "term_id": "GO:0140912",
  "term_label": "membrane destabilizing activity",
  "gene_name": "Defensin beta 118",
  "gene": "UniProtKB:Q96PH6"
}